{
  "gene_name": "Serine_arginine repetitive matrix protein 5",
  "gene_symbol": "SRRM5",
  "gene": "UniProtKB:B3KS81",
  "term_id": "UNKNOWN:0001",
  "term_label": "Unknown molecular function"
}